{
  "gene_symbol": "GBX2",
  "term_label": "RNA polymerase II transcription regulatory region sequence-specific DNA binding",
  "gene": "UniProtKB:P52951",
  "term_id": "GO:0000977",
  "gene_name": "Homeobox protein GBX-2"
}